{
  "gene": "UniProtKB:Q6P1A2",
  "term_id": "GO:0036152",
  "term_label": "phosphatidylethanolamine acyl-chain remodeling",
  "gene_name": "Lysophospholipid acyltransferase 5",
  "gene_symbol": "LPCAT3"
}